{
  "gene_name": "Nuclear receptor subfamily 1 group D member 1",
  "term_label": "response to leptin",
  "gene_symbol": "NR1D1",
  "gene": "UniProtKB:P20393",
  "term_id": "GO:0044321"
}